{
  "gene_name": "Synaptic vesicle glycoprotein 2B",
  "term_id": "GO:0030672",
  "term_label": "synaptic vesicle membrane",
  "gene_symbol": "SV2B",
  "gene": "UniProtKB:Q7L1I2"
}